{
  "term_id": "GO:0004879",
  "term_label": "nuclear receptor activity",
  "gene_name": "Nuclear receptor subfamily 2 group E member 1",
  "gene": "UniProtKB:Q9Y466",
  "gene_symbol": "NR2E1"
}